viral scaffold [GO:0046806] (cellular component) Definition: A complex of proteins that form a scaffold around which the viral capsid is constructed. Relationships: is_a protein-containing complex [GO:0032991]; is part of GO:0019028 Sources: ISBN:0072370319